{
  "gene_name": "Transcriptional regulator QRICH1",
  "gene": "UniProtKB:Q2TAL8",
  "gene_symbol": "QRICH1",
  "term_label": "Unknown biological process",
  "term_id": "UNKNOWN:0002"
}